{
  "gene": "UniProtKB:Q9NP91",
  "gene_name": "Sodium- and chloride-dependent transporter XTRP3",
  "gene_symbol": "SLC6A20",
  "term_id": "GO:0016324",
  "term_label": "apical plasma membrane"
}